{
  "term_label": "plasma membrane",
  "term_id": "GO:0005886",
  "gene_symbol": "LHFPL4",
  "gene_name": "LHFPL tetraspan subfamily member 4 protein",
  "gene": "UniProtKB:Q7Z7J7"
}